{
  "gene_symbol": "COL6A6",
  "term_id": "GO:0031012",
  "gene_name": "Collagen alpha-6(VI) chain",
  "term_label": "extracellular matrix",
  "gene": "UniProtKB:A6NMZ7"
}